L-methionine biosynthetic process from L-homoserine via O-phospho-L-homoserine and cystathionine [GO:0019283] (biological process) Definition: he chemical reactions and pathways resulting in the formation of L-methionine from L-homoserine, via the intermediates O-phospho-L-homoserine and cystathionine. Sources: GOC:go_curators, MetaCyc:PWY-702 Also known as: L-methionine formation from O-phospho-L-homoserine and cystathionine, L-methionine synthesis from O-phospho-L-homoserine and cystathionine, methionine biosynthetic process from O-phospho-L-homoserine and cystathionine Relationships: is a type of modified amino acid metabolic process [GO:0006575]; is a type of GO:0006796; is a type of organophosphate metabolic process [GO:0019637]; is a type of GO:0071266; is a type of GO:0170041